{
  "gene": "UniProtKB:Q8NC60",
  "gene_symbol": "NOA1",
  "term_id": "GO:0007005",
  "gene_name": "Nitric oxide-associated protein 1",
  "term_label": "mitochondrion organization"
}